{
  "gene": "UniProtKB:Q8IWW6",
  "term_label": "plasma membrane",
  "term_id": "GO:0005886",
  "gene_name": "Rho GTPase-activating protein 12",
  "gene_symbol": "ARHGAP12"
}